amidine-lyase activity [GO:0016842] (molecular function) Sources: GOC:krc Relationships: is a type of carbon-nitrogen lyase activity [GO:0016840] Definition: Catalysis of the release of amides or amidines by the cleavage of a carbon-nitrogen bond or the reverse reaction with an amide or amidine as a substrate. Subtypes: GO:0003839, GO:0004018, argininosuccinate lyase activity [GO:0004056], peptidylamidoglycolate lyase activity [GO:0004598], purine imidazole-ring cyclase activity [GO:0050230], ureidoglycolate lyase activity [GO:0050385], glutathione specific gamma-glutamylcyclotransferase activity [GO:0061928], gamma-glutamylaminecyclotransferase activity [GO:0061929], (S)-2-(5-amino-1-(5-phospho-D-ribosyl)imidazole-4-carboxamido) succinate lyase (fumarate-forming) activity [GO:0070626]